{
  "term_label": "NuA4 histone acetyltransferase complex",
  "gene_symbol": "MORF4L2",
  "term_id": "GO:0035267",
  "gene": "UniProtKB:Q15014",
  "gene_name": "Mortality factor 4-like protein 2"
}